{
  "term_id": "UNKNOWN:0001",
  "gene": "UniProtKB:Q96KS9",
  "gene_name": "Protein FAM167A",
  "term_label": "Unknown molecular function",
  "gene_symbol": "FAM167A"
}